{
  "gene": "UniProtKB:Q9H1Q7",
  "term_id": "UNKNOWN:0002",
  "term_label": "Unknown biological process",
  "gene_symbol": "PCED1A",
  "gene_name": "PC-esterase domain-containing protein 1A"
}